{
  "term_id": "GO:0046330",
  "term_label": "positive regulation of JNK cascade",
  "gene": "UniProtKB:O60336",
  "gene_symbol": "MAPKBP1",
  "gene_name": "Mitogen-activated protein kinase-binding protein 1"
}